{
  "term_label": "mRNA binding",
  "term_id": "GO:0003729",
  "gene_symbol": "NCBP3",
  "gene": "UniProtKB:Q53F19",
  "gene_name": "Nuclear cap-binding protein subunit 3"
}